{
  "term_id": "GO:0030003",
  "gene_name": "Zinc transporter ZIP12",
  "term_label": "intracellular monoatomic cation homeostasis",
  "gene": "UniProtKB:Q504Y0",
  "gene_symbol": "SLC39A12"
}